{
  "gene_name": "Carbohydrate sulfotransferase 1",
  "gene": "UniProtKB:O43916",
  "term_id": "GO:0042339",
  "gene_symbol": "CHST1",
  "term_label": "keratan sulfate proteoglycan metabolic process"
}